{
  "gene": "UniProtKB:P02654",
  "gene_symbol": "APOC1",
  "term_id": "GO:0006641",
  "term_label": "triglyceride metabolic process",
  "gene_name": "Apolipoprotein C-I"
}